15-hydroxyprostaglandin-D dehydrogenase (NADP+) activity [GO:0047020] (molecular function) Definition: Catalysis of the reaction: NADP+ + (5Z,13E)-(15S)-9-alpha,15-dihydroxy-11-oxoprosta-5,13-dienoate = NADPH + H+ + (5Z,13E)-9-alpha-hydroxy-11,15-dioxoprosta-5,13-dienoate. Also known as: NADP-dependent 15-hydroxyprostaglandin dehydrogenase, NADP-linked 15-hydroxyprostaglandin dehydrogenase, NADP-specific 15-hydroxyprostaglandin dehydrogenase, (5Z,13E)-(15S)-9alpha,15-dihydroxy-11-oxoprosta-5,13-dienoate:NADP+ 15-oxidoreductase activity, 15-hydroxy PGD2 dehydrogenase activity, 15-hydroxyprostaglandin dehydrogenase (NADP), NADP-PGD2 dehydrogenase activity, NADP-linked prostaglandin D2 dehydrogenase activity, dehydrogenase, 15-hydroxyprostaglandin (nicotinamide adenine dinucleotide phosphate), dehydrogenase, prostaglandin D2, prostaglandin D2 dehydrogenase activity, prostaglandin-D 15-dehydrogenase (NADP(+)) activity, prostaglandin-D 15-dehydrogenase (NADP), prostaglandin-D 15-dehydrogenase (NADP+) activity Sources: EC:1.1.1.196, MetaCyc:1.1.1.196-RXN Relationships: is a type of oxidoreductase activity, acting on the CH-OH group of donors, NAD or NADP as acceptor [GO:0016616]